{
  "gene": "UniProtKB:Q6ZUF6",
  "term_label": "Unknown molecular function",
  "gene_symbol": "LINC00336",
  "term_id": "UNKNOWN:0001",
  "gene_name": "Putative uncharacterized protein encoded by LINC00336"
}